{
  "gene_name": "TGF-beta-activated kinase 1 and MAP3K7-binding protein 2",
  "gene_symbol": "TAB2",
  "gene": "UniProtKB:Q9NYJ8",
  "term_label": "positive regulation of canonical NF-kappaB signal transduction",
  "term_id": "GO:0043123"
}